beta-alanine catabolic process to mevalonate semialdehyde, by transamination [GO:0019486] (biological process) Relationships: is a type of beta-alanine catabolic process [GO:0019484] Sources: GOC:go_curators Definition: The chemical reactions and pathways resulting in the breakdown of beta-alanine into other compounds, including mevalonate semialdehyde, by transamination. Also known as: beta-alanine breakdown to mevalonate semialdehyde, by transamination, beta-alanine degradation to mevalonate semialdehyde, by transamination